glycine decarboxylation via glycine cleavage system [GO:0019464] (biological process) Also known as: glycine cleavage system Relationships: is a type of glycine catabolic process [GO:0006546] Definition: The chemical reactions and pathways resulting in the breakdown of glycine by oxidative cleavage to carbon dioxide, ammonia, and a methylene group, mediated by enzymes of the glycine cleavage complex. Sources: MetaCyc:GLYCLEAV-PWY